{
  "gene": "UniProtKB:A0A1B0GU29",
  "gene_name": "Small integral membrane protein 28",
  "gene_symbol": "SMIM28",
  "term_id": "UNKNOWN:0003",
  "term_label": "Unknown cellular component"
}